{
  "term_id": "UNKNOWN:0002",
  "gene_name": "F-box only protein 41",
  "term_label": "Unknown biological process",
  "gene_symbol": "FBXO41",
  "gene": "UniProtKB:Q8TF61"
}